{
  "term_id": "GO:0000956",
  "gene": "UniProtKB:Q9H0D6",
  "term_label": "nuclear-transcribed mRNA catabolic process",
  "gene_symbol": "XRN2",
  "gene_name": "5'-3' exoribonuclease 2"
}